{
  "gene_name": "T cell receptor alpha variable 2",
  "gene": "UniProtKB:A0A0B4J234",
  "term_id": "UNKNOWN:0001",
  "gene_symbol": "TRAV2",
  "term_label": "Unknown molecular function"
}